{
  "gene_name": "Death domain-associated protein 6",
  "gene_symbol": "DAXX",
  "term_label": "negative regulation of DNA-templated transcription",
  "term_id": "GO:0045892",
  "gene": "UniProtKB:Q9UER7"
}